SAGA complex localization to transcription regulatory region [GO:0072742] (biological process) Sources: GOC:mah Relationships: is a type of protein-containing complex localization [GO:0031503] Also known as: SAGA complex localization to promoter, SAGA complex recruitment Definition: Any process in which a SAGA complex is transported to, or maintained in, a specific location in the transcription regulatory region of a gene.